{
  "gene": "UniProtKB:O14795",
  "term_label": "syntaxin-1 binding",
  "term_id": "GO:0017075",
  "gene_name": "Protein unc-13 homolog B",
  "gene_symbol": "UNC13B"
}